{
  "term_id": "GO:0007204",
  "term_label": "positive regulation of cytosolic calcium ion concentration",
  "gene_symbol": "CCR9",
  "gene": "UniProtKB:P51686",
  "gene_name": "C-C chemokine receptor type 9"
}